serine 3-dehydrogenase activity [GO:0031132] (molecular function) Relationships: is a type of oxidoreductase activity, acting on the CH-OH group of donors, NAD or NADP as acceptor [GO:0016616] Also known as: L-serine:NADP+ 3-oxidoreductase activity Definition: Catalysis of the reaction: L-serine + NADP+ = L-alpha-formylglycine + 2 H+ + NADPH. Sources: EC:1.1.1.276, RHEA:21596